{
  "gene_name": "Ephrin type-A receptor 2",
  "term_id": "GO:0004714",
  "term_label": "transmembrane receptor protein tyrosine kinase activity",
  "gene": "UniProtKB:P29317",
  "gene_symbol": "EPHA2"
}